oocyte growth in germarium-derived egg chamber [GO:0030715] (BP) Sources: GOC:mtg_sensu, ISBN:0879694238 Definition: The increase in volume of an oocyte during the growth phase of the egg chamber, once the egg chamber has left the germarium. An example of this process is found in Drosophila melanogaster. Relationships: is a type of oocyte growth [GO:0001555]; is part of GO:0007295